{
  "gene_symbol": "BICC1",
  "term_id": "UNKNOWN:0001",
  "term_label": "Unknown molecular function",
  "gene": "UniProtKB:Q9H694",
  "gene_name": "Protein bicaudal C homolog 1"
}